response to wounding [GO:0009611] (biological process) Definition: Any process that results in a change in state or activity of a cell or an organism (in terms of movement, secretion, enzyme production, gene expression, etc.) as a result of a stimulus indicating damage to the organism. Regulation: regulated by GO:1903034; negatively regulated by negative regulation of response to wounding [GO:1903035]; positively regulated by GO:1903036 Relationships: is a type of response to stress [GO:0006950] Also known as: physiological response to wounding Sources: GOC:go_curators Subtypes: GO:0002210, jasmonic acid and ethylene-dependent systemic resistance [GO:0009861], GO:0014822, response to injury involved in regulation of muscle adaptation [GO:0014876], wound healing [GO:0042060], GO:0048678, inflammatory response to wounding [GO:0090594]